{
  "gene_symbol": "THRB",
  "gene_name": "Thyroid hormone receptor beta",
  "term_id": "GO:0000978",
  "term_label": "RNA polymerase II cis-regulatory region sequence-specific DNA binding",
  "gene": "UniProtKB:P10828"
}